negative regulation of T cell differentiation [GO:0045581] (biological process) Relationships: is a type of regulation of T cell differentiation [GO:0045580]; is a type of negative regulation of lymphocyte differentiation [GO:0045620]; is a type of GO:0050868; RO_0002212 T cell differentiation [GO:0030217] Definition: Any process that stops, prevents, or reduces the frequency, rate or extent of T cell differentiation. Sources: GOC:go_curators Also known as: down regulation of T cell differentiation, down-regulation of T cell differentiation, downregulation of T cell differentiation, negative regulation of T lymphocyte differentiation, negative regulation of T-cell differentiation, negative regulation of T-lymphocyte differentiation, inhibition of T cell differentiation, negative regulation of T cell development Subtypes: negative regulation of T cell differentiation in thymus [GO:0033085], negative regulation of extrathymic T cell differentiation [GO:0033086], negative regulation of memory T cell differentiation [GO:0043381], negative regulation of cytotoxic T cell differentiation [GO:0045584], negative regulation of gamma-delta T cell differentiation [GO:0045587], negative regulation of regulatory T cell differentiation [GO:0045590], negative regulation of alpha-beta T cell differentiation [GO:0046639], negative regulation of pro-T cell differentiation [GO:2000175] Note: Note that immunologists typically use the word 'development' to refer to cells of B or T cell lineages undergoing the process that GO describes as 'cell differentiation'.